regulation of L-leucine biosynthetic process [GO:2001276] (biological process) Sources: GOC:obol Subtypes: negative regulation of L-leucine biosynthetic process [GO:2001277], GO:2001278 Also known as: regulation of leucine biosynthetic process, regulation of L-leucine anabolism, regulation of L-leucine biosynthesis, regulation of L-leucine formation, regulation of L-leucine synthesis Relationships: is a type of regulation of small molecule metabolic process [GO:0062012]; is a type of regulation of amino acid biosynthetic process [GO:2000282]; regulates GO:0009098 Definition: Any process that modulates the frequency, rate or extent of L-leucine biosynthetic process.